stigma papilla [GO:0090397] (CC) Definition: A plant cell papilla that is part of a stigma papilla cell. Sources: GOC:tb Note: Part of stigma papilla cell (PO:0025168). Relationships: is a type of plant cell papilla [GO:0090395]